response to glucagon [GO:0033762] (biological process) Also known as: response to glucagon stimulus Sources: GOC:sl Definition: Any process that results in a change in state or activity of a cell or an organism (in terms of movement, secretion, enzyme production, gene expression, etc.) as a result of a glucagon stimulus. Subtypes: cellular response to glucagon stimulus [GO:0071377] Relationships: is a type of response to peptide hormone [GO:0043434]